{
  "term_label": "intracellular sodium ion homeostasis",
  "gene": "UniProtKB:P14415",
  "gene_name": "Sodium_potassium-transporting ATPase subunit beta-2",
  "gene_symbol": "ATP1B2",
  "term_id": "GO:0006883"
}